{
  "gene": "UniProtKB:P31146",
  "term_label": "actin filament organization",
  "term_id": "GO:0007015",
  "gene_symbol": "CORO1A",
  "gene_name": "Coronin-1A"
}